{
  "gene": "UniProtKB:Q9Y3L3",
  "gene_name": "SH3 domain-binding protein 1",
  "gene_symbol": "SH3BP1",
  "term_label": "regulation of Rac protein signal transduction",
  "term_id": "GO:0035020"
}